{
  "term_label": "cilium assembly",
  "term_id": "GO:0060271",
  "gene_symbol": "CEP89",
  "gene_name": "Centrosomal protein of 89 kDa",
  "gene": "UniProtKB:Q96ST8"
}